{
  "gene_name": "Forkhead box protein D4-like 1",
  "gene_symbol": "FOXD4L1",
  "term_id": "GO:0000978",
  "term_label": "RNA polymerase II cis-regulatory region sequence-specific DNA binding",
  "gene": "UniProtKB:Q9NU39"
}